{
  "gene_symbol": "KRT28",
  "term_id": "GO:0045109",
  "gene_name": "Keratin, type I cytoskeletal 28",
  "gene": "UniProtKB:Q7Z3Y7",
  "term_label": "intermediate filament organization"
}